response to cation stress [GO:0043157] (biological process) Relationships: is a type of GO:0009651 References: PMID:14762213 Sources: GOC:jl Definition: Any process that results in a change in state or activity of a cell or an organism (in terms of movement, secretion, enzyme production, gene expression, etc.) as a result of cation stress, an increase or decrease in the concentration of positively charged ions in the environment. Subtypes: cellular response to cation stress [GO:0071473]